{
  "gene_symbol": "IDH1",
  "term_label": "peroxisome",
  "gene": "UniProtKB:O75874",
  "gene_name": "Isocitrate dehydrogenase [NADP] cytoplasmic",
  "term_id": "GO:0005777"
}